chiasma [GO:0005712] (cellular component) Sources: ISBN:0198506732 Relationships: is a type of cellular anatomical structure [GO:0110165]; is part of condensed nuclear chromosome [GO:0000794] Definition: A connection formed between chromatids, visible during meiosis, thought to be the point of the interchange involved in crossing-over.